cellular response to hormone stimulus [GO:0032870] (biological process) Definition: Any process that results in a change in state or activity of a cell (in terms of movement, secretion, enzyme production, gene expression, etc.) as a result of a hormone stimulus. Subtypes: GO:0044320, GO:0071215, cellular response to auxin stimulus [GO:0071365], cellular response to brassinosteroid stimulus [GO:0071367], cellular response to cytokinin stimulus [GO:0071368], cellular response to ethylene stimulus [GO:0071369], cellular response to gibberellin stimulus [GO:0071370], cellular response to gonadotropin stimulus [GO:0071371], GO:0071374, cellular response to peptide hormone stimulus [GO:0071375], cellular response to prostaglandin stimulus [GO:0071379], cellular response to steroid hormone stimulus [GO:0071383], cellular response to estrogen stimulus [GO:0071391], cellular response to jasmonic acid stimulus [GO:0071395], cellular response to thyroid hormone stimulus [GO:0097067] Sources: GOC:mah Relationships: is a type of response to hormone [GO:0009725]; is a type of GO:0070887; is a type of cellular response to endogenous stimulus [GO:0071495]